{
  "gene_name": "C-Jun-amino-terminal kinase-interacting protein 3",
  "term_label": "kinesin binding",
  "gene_symbol": "MAPK8IP3",
  "term_id": "GO:0019894",
  "gene": "UniProtKB:Q9UPT6"
}